{
  "term_id": "UNKNOWN:0003",
  "gene": "UniProtKB:A2RU48",
  "gene_symbol": "SMCO3",
  "term_label": "Unknown cellular component",
  "gene_name": "Single-pass membrane and coiled-coil domain-containing protein 3"
}